{
  "gene": "UniProtKB:Q7L8C5",
  "gene_symbol": "SYT13",
  "term_id": "GO:0017158",
  "term_label": "regulation of calcium ion-dependent exocytosis",
  "gene_name": "Synaptotagmin-13"
}